host cell plasma membrane [GO:0020002] (cellular component) Definition: The plasma membrane surrounding a host cell. Sources: GOC:mb Relationships: is_a host cell membrane [GO:0033644]